{
  "term_id": "GO:0031514",
  "gene": "UniProtKB:Q8IY82",
  "term_label": "motile cilium",
  "gene_symbol": "DRC7",
  "gene_name": "Dynein regulatory complex subunit 7"
}